alphaIIb-beta3 integrin-CD9-CD47-platelet glycoprotein Ib complex [GO:0071086] (CC) Relationships: is a type of glycoprotein complex [GO:0090665]; is a type of GO:0098797 References: PMID:10429193 Also known as: ITGA2b-ITGB3-CD9-GP1b-CD47 complex Definition: A protein complex that consists of an alphaIIb-beta3 integrin complex bound to the cell surface proteins CD9 and CD47, and the heterodimeric platelet glycoprotein Ib.